{
  "term_label": "exogenous lipid antigen binding",
  "gene": "UniProtKB:P29016",
  "gene_symbol": "CD1B",
  "term_id": "GO:0030884",
  "gene_name": "T-cell surface glycoprotein CD1b"
}